{
  "gene_symbol": "NAT10",
  "term_id": "GO:0051391",
  "gene": "UniProtKB:Q9H0A0",
  "gene_name": "RNA cytidine acetyltransferase",
  "term_label": "tRNA acetylation"
}